bisphosphoglycerate 3-phosphatase activity [GO:0034417] (molecular function) Also known as: 2,3-bisphospho-D-glycerate 3-phosphohydrolase activity Definition: Catalysis of the reaction: (2R)-2,3-bisphosphoglycerate + H2O = (2R)-2-phosphoglycerate + phosphate. Relationships: is a type of GO:0016791 References: PMID:18413611 Sources: GOC:mah, RHEA:27381